{
  "term_label": "regulation of transcription by RNA polymerase II",
  "gene": "UniProtKB:Q33E94",
  "term_id": "GO:0006357",
  "gene_symbol": "RFX4",
  "gene_name": "Transcription factor RFX4"
}